{
  "gene": "UniProtKB:Q969Q0",
  "term_label": "cytosolic large ribosomal subunit",
  "gene_symbol": "RPL36AL",
  "gene_name": "Ribosomal protein eL42-like",
  "term_id": "GO:0022625"
}